{
  "term_id": "GO:0005109",
  "gene": "UniProtKB:Q93097",
  "gene_symbol": "WNT2B",
  "gene_name": "Protein Wnt-2b",
  "term_label": "frizzled binding"
}